negative regulation of cardiac muscle cell apoptotic process [GO:0010667] (biological process) Also known as: down regulation of cardiac muscle cell apoptosis, down-regulation of cardiac muscle cell apoptosis, downregulation of cardiac muscle cell apoptosis, inhibition of cardiac muscle cell apoptosis, negative regulation of cardiac muscle cell apoptosis Definition: Any process that decreases the rate or extent of cardiac cell apoptotic process, a form of programmed cell death induced by external or internal signals that trigger the activity of proteolytic caspases whose actions dismantle a cardiac muscle cell and result in its death. Relationships: is a type of negative regulation of striated muscle cell apoptotic process [GO:0010664]; is a type of GO:0010665; negatively regulates cardiac muscle cell apoptotic process [GO:0010659] Sources: GOC:BHF, GOC:dph, GOC:mtg_apoptosis, GOC:rl, GOC:tb